nucleoside diphosphate phosphatase activity [GO:0017110] (MF) Relationships: is a type of pyrophosphatase activity [GO:0016462] Subtypes: GDP phosphatase activity [GO:0004382], CDP phosphatase activity [GO:0036384], ADP phosphatase activity [GO:0043262], 8-oxo-dGDP phosphatase activity [GO:0044715], GO:0044716, 8-hydroxy-dADP phosphatase activity [GO:0044717], UDP phosphatase activity [GO:0045134], dIDP phosphatase activity [GO:0097383], 8-oxo-dADP diphosphate phosphatase activity [GO:0102459], IDP phosphatase activity [GO:1990003] Also known as: apyrase activity, nucleoside diphosphatase activity, nucleoside-diphosphatase activity, inosine 5'-diphosphatase, inosine diphosphatase, type B nucleoside diphosphatase, type L nucleoside diphosphatase, NDPase activity, nucleoside 5'-diphosphatase activity, nucleoside diphosphate phosphohydrolase activity, nucleoside-diphosphate phosphohydrolase activity Definition: Catalysis of the reaction: a nucleoside diphosphate + H2O = a nucleoside monophosphate + phosphate. Sources: EC:3.6.1.6